{
  "term_id": "GO:0051965",
  "gene_name": "SLIT and NTRK-like protein 3",
  "gene_symbol": "SLITRK3",
  "term_label": "positive regulation of synapse assembly",
  "gene": "UniProtKB:O94933"
}